{
  "term_label": "Unknown biological process",
  "gene_name": "Tuberoinfundibular peptide of 39 residues",
  "gene_symbol": "PTH2",
  "term_id": "UNKNOWN:0002",
  "gene": "UniProtKB:Q96A98"
}